diaphragm contraction [GO:0002086] (biological process) Definition: A process in which force is generated within involuntary skeletal muscle tissue, resulting in a change in muscle geometry. This process occurs in the diaphragm. Force generation involves a chemo-mechanical energy conversion step that is carried out by the actin/myosin complex activity, which generates force through ATP hydrolysis. The diaphragm is a striated muscle that is necessary for the process of respiratory gaseous exchange. References: PMID:12458206 Sources: GOC:dph, GOC:mtg_muscle Relationships: is a type of involuntary skeletal muscle contraction [GO:0003011]; is a type of respiratory system process [GO:0003016]